{
  "term_id": "GO:0043252",
  "gene_name": "Solute carrier organic anion transporter family member 1C1",
  "gene": "UniProtKB:Q9NYB5",
  "gene_symbol": "SLCO1C1",
  "term_label": "sodium-independent organic anion transport"
}